{
  "term_id": "GO:0045236",
  "gene_name": "C-C motif chemokine 27",
  "gene": "UniProtKB:Q9Y4X3",
  "gene_symbol": "CCL27",
  "term_label": "CXCR chemokine receptor binding"
}